{
  "term_label": "regulation of transcription by RNA polymerase II",
  "term_id": "GO:0006357",
  "gene_symbol": "HMX1",
  "gene": "UniProtKB:Q9NP08",
  "gene_name": "Homeobox protein HMX1"
}